isocitrate epimerase activity [GO:0047755] (MF) Definition: Catalysis of the reaction: D-threo-isocitrate = D-erythro-isocitrate. Sources: EC:5.1.2.6, RHEA:10820 Also known as: (1R,2S)-1-hydroxypropane-1,2,3-tricarboxylate 1-epimerase activity Relationships: is a type of racemase and epimerase activity, acting on hydroxy acids and derivatives [GO:0016856]